{
  "term_id": "GO:0005886",
  "gene_name": "Thrombospondin type-1 domain-containing protein 7A",
  "gene": "UniProtKB:Q9UPZ6",
  "term_label": "plasma membrane",
  "gene_symbol": "THSD7A"
}